negative regulation of glutathione biosynthetic process [GO:1903787] (biological process) Also known as: down regulation of glutathione anabolism, down regulation of glutathione biosynthesis, down regulation of glutathione biosynthetic process, down regulation of glutathione formation, down regulation of glutathione synthesis, down-regulation of glutathione anabolism, down-regulation of glutathione biosynthesis, down-regulation of glutathione biosynthetic process, down-regulation of glutathione formation, down-regulation of glutathione synthesis, downregulation of glutathione anabolism, downregulation of glutathione biosynthesis, downregulation of glutathione biosynthetic process, downregulation of glutathione formation, downregulation of glutathione synthesis, negative regulation of glutathione anabolism, negative regulation of glutathione biosynthesis, negative regulation of glutathione formation, negative regulation of glutathione synthesis, inhibition of glutathione anabolism, inhibition of glutathione biosynthesis, inhibition of glutathione biosynthetic process, inhibition of glutathione formation, inhibition of glutathione synthesis Sources: GOC:PARL, GOC:TermGenie, GOC:bf, GO_REF:0000058 Relationships: is a type of negative regulation of biosynthetic process [GO:0009890]; is a type of GO:0034249; is a type of regulation of glutathione biosynthetic process [GO:1903786]; negatively regulates glutathione biosynthetic process [GO:0006750] Definition: Any process that stops, prevents or reduces the frequency, rate or extent of glutathione biosynthetic process.